{
  "gene": "UniProtKB:Q6IV72",
  "gene_symbol": "ZNF425",
  "gene_name": "Zinc finger protein 425",
  "term_label": "nucleus",
  "term_id": "GO:0005634"
}